{
  "term_label": "regulation of gene expression",
  "term_id": "GO:0010468",
  "gene": "UniProtKB:Q8TD26",
  "gene_name": "Chromodomain-helicase-DNA-binding protein 6",
  "gene_symbol": "CHD6"
}